{
  "term_label": "immune response",
  "gene_symbol": "MARCHF8",
  "term_id": "GO:0006955",
  "gene": "UniProtKB:Q5T0T0",
  "gene_name": "E3 ubiquitin-protein ligase MARCHF8"
}